{
  "gene": "UniProtKB:Q01101",
  "term_id": "GO:0000978",
  "gene_name": "Insulinoma-associated protein 1",
  "term_label": "RNA polymerase II cis-regulatory region sequence-specific DNA binding",
  "gene_symbol": "INSM1"
}